{
  "gene": "UniProtKB:Q9P0W0",
  "term_label": "T cell activation involved in immune response",
  "gene_symbol": "IFNK",
  "term_id": "GO:0002286",
  "gene_name": "Interferon kappa"
}